{
  "term_id": "GO:0003677",
  "term_label": "DNA binding",
  "gene": "UniProtKB:Q68CP9",
  "gene_symbol": "ARID2",
  "gene_name": "AT-rich interactive domain-containing protein 2"
}